{
  "gene": "UniProtKB:Q04828",
  "gene_name": "Aldo-keto reductase family 1 member C1",
  "gene_symbol": "AKR1C1",
  "term_label": "ketosteroid monooxygenase activity",
  "term_id": "GO:0047086"
}